{
  "term_id": "GO:0030674",
  "gene_name": "Integrator complex subunit 6",
  "gene_symbol": "INTS6",
  "gene": "UniProtKB:Q9UL03",
  "term_label": "protein-macromolecule adaptor activity"
}